{
  "term_label": "positive regulation of transcription by RNA polymerase II",
  "gene": "UniProtKB:P40424",
  "gene_name": "Pre-B-cell leukemia transcription factor 1",
  "term_id": "GO:0045944",
  "gene_symbol": "PBX1"
}